{
  "gene": "UniProtKB:A0A8V8TMC4",
  "gene_symbol": "CCNYL1B",
  "term_id": "GO:0005886",
  "gene_name": "Cyclin N-terminal domain-containing protein",
  "term_label": "plasma membrane"
}